{
  "term_label": "Unknown molecular function",
  "gene_name": "G patch domain-containing protein 2-like",
  "gene_symbol": "GPATCH2L",
  "term_id": "UNKNOWN:0001",
  "gene": "UniProtKB:Q9NWQ4"
}